biogenic amine metabolic process [GO:0006576] (BP) Definition: The chemical reactions and pathways occurring at the level of individual cells involving any of a group of naturally occurring, biologically active amines, such as norepinephrine, histamine, and serotonin, many of which act as neurotransmitters. Also known as: biogenic amine metabolism, cellular biogenic amine metabolic process Sources: GOC:jl, ISBN:0395825172 Subtypes: GO:0001692, GO:0006584, polyamine metabolic process [GO:0006595], biogenic amine biosynthetic process [GO:0042401], phenylethylamine metabolic process [GO:0042443] Relationships: is a type of GO:0009308